{
  "gene_name": "Host cell factor C1 regulator 1",
  "gene_symbol": "HCFC1R1",
  "term_id": "UNKNOWN:0001",
  "term_label": "Unknown molecular function",
  "gene": "UniProtKB:Q9NWW0"
}